aldarate transmembrane transport [GO:0042869] (biological process) Relationships: is a type of dicarboxylic acid transport [GO:0006835]; is a type of carboxylic acid transmembrane transport [GO:1905039] Subtypes: D-glucarate transmembrane transport [GO:0042870], GO:1902300 Definition: The process in which aldarate is transported across a lipid bilayer, from one side of a membrane to the other. Also known as: aldarate transport Sources: GOC:go_curators